protein localization to membrane raft [GO:1903044] (biological process) Subtypes: GO:0032596, protein localization to plasma membrane raft [GO:0044860] Definition: A process in which a protein is transported to, or maintained in, a location within a membrane raft. Relationships: is a type of protein localization to membrane [GO:0072657] Also known as: protein localisation in membrane raft, protein localisation to membrane raft, protein localization in membrane raft References: PMID:19414744 Sources: GOC:TermGenie, GOC:dl, GO_REF:0000087